4-galactosyl-N-acetylglucosaminide 3-alpha-L-fucosyltransferase activity [GO:0017083] (molecular function) Definition: Catalysis of the reaction: GDP-beta-L-fucose + beta-D-galactosyl-(1,4)-N-acetyl-D-glucosaminyl-R = GDP + 1,4-beta-D-galactosyl-(1,4)-[alpha-L-fucosyl-(1,3)]-N-acetyl-D-glucosaminyl-R. Sources: EC:2.4.1.152, RHEA:14257 Also known as: galactoside 3-L-fucosyltransferase activity, Lewis-negative alpha-3-fucosyltransferase activity, plasma alpha-3-fucosyltransferase activity, GDP-L-fucose:1,4-beta-D-galactosyl-N-acetyl-D-glucosaminyl-R 3-L-fucosyltransferase activity, GDP-beta-L-fucose:1,4-beta-D-galactosyl-N-acetyl-D-glucosaminyl-R 3-L-fucosyltransferase activity, GDP-beta-L-fucose:1,4-beta-D-galactosyl-N-acetyl-D-glucosaminyl-R 3-alpha-L-fucosyltransferase activity, galactoside 3-fucosyltransferase activity, guanosine diphosphofucose-glucoside alpha-1->3-fucosyltransferase activity, guanosine diphosphofucose-glucoside alpha1->3-fucosyltransferase activity Relationships: is_a alpha-(1->3)-fucosyltransferase activity [GO:0046920]